{
  "term_label": "Notch signaling pathway",
  "term_id": "GO:0007219",
  "gene": "UniProtKB:Q9Y5J3",
  "gene_name": "Hairy_enhancer-of-split related with YRPW motif protein 1",
  "gene_symbol": "HEY1"
}